{
  "gene": "UniProtKB:P84095",
  "gene_symbol": "RHOG",
  "term_label": "cell projection",
  "term_id": "GO:0042995",
  "gene_name": "Rho-related GTP-binding protein RhoG"
}